negative regulation of osteoclast development [GO:2001205] (biological process) Relationships: is a type of GO:0045671; is a type of GO:2001204; RO_0002212 osteoclast development [GO:0036035] Definition: Any process that stops, prevents or reduces the frequency, rate or extent of osteoclast development. Also known as: negative regulation of osteoclast cell development Sources: GOC:obol